{
  "term_label": "plasma membrane",
  "term_id": "GO:0005886",
  "gene_name": "ER membrane protein complex subunit 5",
  "gene_symbol": "MMGT1",
  "gene": "UniProtKB:Q8N4V1"
}